{
  "gene_symbol": "FCGR1A",
  "term_id": "GO:0007166",
  "term_label": "cell surface receptor signaling pathway",
  "gene_name": "High affinity immunoglobulin gamma Fc receptor I",
  "gene": "UniProtKB:P12314"
}